hydrolase activity, acting on acid carbon-carbon bonds, in ketonic substances [GO:0016823] (molecular function) Definition: Catalysis of the hydrolysis of any acid carbon-carbon bond in a ketonic substance, a substance containing a keto (C=O) group. Sources: EC:3.7.1.- Relationships: is a type of hydrolase activity, acting on acid carbon-carbon bonds [GO:0016822] Subtypes: fumarylacetoacetase activity [GO:0004334], 2-hydroxy-6-oxohepta-2,4-dienoate hydrolase activity [GO:0018765], dihydrophloroglucinol hydrolase activity [GO:0018766], 2-hydroxy-6-oxo-6-(2'-aminophenyl)hexa-2,4-dienoate hydrolase activity [GO:0018768], 2-hydroxy-6-oxonona-2,4-dienedioate hydrolase activity [GO:0018771], GO:0018772, acetylpyruvate hydrolase activity [GO:0018773], 2,6-dioxo-6-phenylhexa-3-enoate hydrolase activity [GO:0018774], 2-hydroxymuconate-semialdehyde hydrolase activity [GO:0018775], kynureninase activity [GO:0030429], GO:0030603, fumarylpyruvate hydrolase activity [GO:0034545], cobalt-precorrin-5A acetaldehyde-lyase activity [GO:0043779], GO:0047621, GO:0047699, cyclohexane-1,3-dione hydrolase activity [GO:0047796], phloretin hydrolase activity [GO:0050180], 2-hydroxy-6-oxonona-2,4,7-trienedioate hydrolase activity [GO:0052823], maleylpyruvate hydrolase activity [GO:0102054], GO:0102296, GO:0102481